Lsm1-7-Pat1 complex [GO:1990726] (CC) References: PMID:19121818, PMID:23620288, PMID:24139796, PMID:27627834, PMID:28768202 Sources: GOC:bhm, GOC:krc Relationships: is a type of Sm-like protein family complex [GO:0120114] Definition: A conserved, heteroheptameric, cytoplasmic protein complex composed of Lsm1, Lsm2, Lsm3, Lsm4, Lsm5, Lsm6, Lsm7, and Pat1, or orthologs thereof, that shows a strong binding preference for oligoadenylated RNAs over polyadenylated RNAs. May bind further associated proteins. Facilitates the deadenylation-dependent decapping of mRNA in the P-body thereby regulating mRNA decay and subsequent degradation by the 5' to 3' pathway.